positive regulation of lysozyme activity [GO:1903592] (biological process) References: PMID:23954697 Sources: GOC:TermGenie, GOC:mr, GO_REF:0000059 Relationships: is a type of positive regulation of hydrolase activity [GO:0051345]; positively regulates lysozyme activity [GO:0003796] Also known as: positive regulation of 1,4-N-acetylmuramidase activity, positive regulation of N,O-diacetylmuramidase activity, positive regulation of mucopeptide N-acetylmuramoylhydrolase activity, positive regulation of mucopeptide glucohydrolase activity, positive regulation of muramidase activity, positive regulation of peptidoglycan N-acetylmuramoylhydrolase activity, up regulation of 1,4-N-acetylmuramidase activity, up regulation of N,O-diacetylmuramidase activity, up regulation of lysozyme activity, up regulation of mucopeptide N-acetylmuramoylhydrolase activity, up regulation of mucopeptide glucohydrolase activity, up regulation of muramidase activity, up regulation of peptidoglycan N-acetylmuramoylhydrolase activity, up-regulation of 1,4-N-acetylmuramidase activity, up-regulation of N,O-diacetylmuramidase activity, up-regulation of lysozyme activity, up-regulation of mucopeptide N-acetylmuramoylhydrolase activity, up-regulation of mucopeptide glucohydrolase activity, up-regulation of muramidase activity, up-regulation of peptidoglycan N-acetylmuramoylhydrolase activity, upregulation of 1,4-N-acetylmuramidase activity, upregulation of N,O-diacetylmuramidase activity, upregulation of lysozyme activity, upregulation of mucopeptide N-acetylmuramoylhydrolase activity, upregulation of mucopeptide glucohydrolase activity, upregulation of muramidase activity, upregulation of peptidoglycan N-acetylmuramoylhydrolase activity, activation of 1,4-N-acetylmuramidase activity, activation of N,O-diacetylmuramidase activity, activation of lysozyme activity, activation of mucopeptide N-acetylmuramoylhydrolase activity, activation of mucopeptide glucohydrolase activity, activation of muramidase activity, activation of peptidoglycan N-acetylmuramoylhydrolase activity, activation of L-7001, activation of PR1-lysozyme, activation of globulin G, activation of globulin G1, activation of lysozyme g, positive regulation of L-7001, positive regulation of PR1-lysozyme, positive regulation of globulin G, positive regulation of globulin G1, positive regulation of lysozyme g, up regulation of L-7001, up regulation of PR1-lysozyme, up regulation of globulin G, up regulation of globulin G1, up regulation of lysozyme g, up-regulation of L-7001, up-regulation of PR1-lysozyme, up-regulation of globulin G, up-regulation of globulin G1, up-regulation of lysozyme g, upregulation of L-7001, upregulation of PR1-lysozyme, upregulation of globulin G, upregulation of globulin G1, upregulation of lysozyme g Definition: Any process that activates or increases the frequency, rate or extent of lysozyme activity.